{
  "gene": "UniProtKB:P51674",
  "term_label": "regulation of filopodium assembly",
  "gene_name": "Neuronal membrane glycoprotein M6-a",
  "term_id": "GO:0051489",
  "gene_symbol": "GPM6A"
}